peptidyl-lysine 3-dioxygenase activity [GO:0106155] (molecular function) References: PMID:29915238 Sources: GOC:al, RHEA:57152 Definition: Catalysis of the reaction: protein L-lysine + 2-oxoglutarate + O2 = protein 3-hydroxy-L-lysine + succinate + CO2. Relationships: is_a 2-oxoglutarate-dependent dioxygenase activity [GO:0016706]; is a type of GO:0140096